{
  "gene_name": "Oxidative stress-responsive serine-rich protein 1",
  "gene": "UniProtKB:Q9NX31",
  "gene_symbol": "OSER1",
  "term_label": "Unknown molecular function",
  "term_id": "UNKNOWN:0001"
}